{
  "gene_name": "Leucine-rich repeat and immunoglobulin-like domain-containing nogo receptor-interacting protein 1",
  "gene": "UniProtKB:Q96FE5",
  "term_id": "GO:0005154",
  "gene_symbol": "LINGO1",
  "term_label": "epidermal growth factor receptor binding"
}